pyrimidine dimer repair by nucleotide-excision repair [GO:0000720] (biological process) Sources: GOC:elh Note: Note that the repair of pyrimidine dimers by nucleotide excision repair involves the same gene products that are involved in general nucleotide excision repair. Consider also annotating to other children of the biological process term 'nucleotide-excision repair ; GO:0006289'. Relationships: is a type of nucleotide-excision repair [GO:0006289]; is a type of pyrimidine dimer repair [GO:0006290] Definition: The repair of UV-induced T-T, C-T, and C-C dimers by the recognition and removal of the damaged DNA strand from the DNA helix as an oligonucleotide. The small gap left in the DNA helix is filled in by the sequential action of DNA polymerase and DNA ligase.